{
  "gene": "UniProtKB:O94817",
  "gene_name": "Ubiquitin-like protein ATG12",
  "term_id": "GO:0019776",
  "term_label": "Atg8-family ligase activity",
  "gene_symbol": "ATG12"
}